proximal straight tubule development [GO:0072020] (biological process) Subtypes: metanephric proximal straight tubule development [GO:0072230] Sources: GOC:mtg_kidney_jan10 Relationships: is a type of nephron tubule development [GO:0072080]; is part of proximal tubule development [GO:0072014] Also known as: S3 development Definition: The process whose specific outcome is the progression of the proximal straight tubule over time, from its formation to the mature structure. The proximal straight tubule is the part of the descending limb that extends from the proximal convoluted tubule to the descending thin tubule.